{
  "gene_symbol": "TBK1",
  "term_id": "GO:0004674",
  "gene": "UniProtKB:Q9UHD2",
  "gene_name": "Serine_threonine-protein kinase TBK1",
  "term_label": "protein serine/threonine kinase activity"
}